{
  "gene": "UniProtKB:P82663",
  "gene_symbol": "MRPS25",
  "term_id": "UNKNOWN:0002",
  "gene_name": "Small ribosomal subunit protein mS25",
  "term_label": "Unknown biological process"
}